{
  "gene": "UniProtKB:Q3LI66",
  "term_id": "UNKNOWN:0001",
  "term_label": "Unknown molecular function",
  "gene_symbol": "KRTAP6-2",
  "gene_name": "Keratin-associated protein 6-2"
}